{
  "gene_name": "Polycystin-2-like protein 2",
  "term_label": "membrane",
  "gene_symbol": "PKD2L2",
  "gene": "UniProtKB:Q9NZM6",
  "term_id": "GO:0016020"
}